antigen processing and presentation of exogenous peptide antigen via MHC class I, TAP-dependent [GO:0002479] (biological process) References: PMID:15224093, PMID:15771591, PMID:16181335 Sources: GOC:add Also known as: cross presentation, cross-presentation, TAP-dependent antigen processing and presentation of exogenous peptide antigen via MHC class I, TAP-dependent exogenous peptide antigen processing and presentation via MHC class I, exogenous peptide antigen processing and presentation via MHC class I, TAP-dependent Relationships: is a type of GO:0042590 Definition: The process in which an antigen-presenting cell expresses a peptide antigen of exogenous origin on its cell surface in association with an MHC class I protein complex following intracellular transport via a TAP (transporter associated with antigen processing) pathway. The peptide is typically a fragment of a larger exogenous protein which has been degraded within the cell and is dependent on TAP transport from the cytosol to ER for association with the MHC class I molecule. Class I here refers to classical class I molecules.